self-resistance to endogenously produced metabolite [GO:0140729] (biological process) References: PMID:21923907, PMID:29763292 Relationships: is a type of detoxification [GO:0098754] Definition: A process that reduces or removes the toxicity of an endogenously produced substance. Mechanisms of resistance to endogenously produced compounds include modification the compound, export, sequestration, or mutations in the target enzyme. Also known as: prevention of self-toxicity, self-resistance to bioactive secondary metabolite, self-resistance to endogenously produced compound, self-resistance to endogenously produced toxin